{
  "term_id": "GO:0005886",
  "term_label": "plasma membrane",
  "gene": "UniProtKB:Q96HJ5",
  "gene_symbol": "MS4A3",
  "gene_name": "Membrane-spanning 4-domains subfamily A member 3"
}